riboflavin biosynthetic process [GO:0009231] (biological process) Definition: The chemical reactions and pathways resulting in the formation of riboflavin (vitamin B2), the precursor for the coenzymes flavin mononucleotide (FMN) and flavin adenine dinucleotide (FAD). Also known as: riboflavin anabolism, riboflavin biosynthesis, riboflavin formation, riboflavin synthesis, vitamin B2 biosynthesis, vitamin B2 biosynthetic process, vitamin G biosynthesis, vitamin G biosynthetic process Relationships: is a type of riboflavin metabolic process [GO:0006771]; is a type of water-soluble vitamin biosynthetic process [GO:0042364]; is a type of flavin-containing compound biosynthetic process [GO:0042727] References: PMID:10940330 Sources: GOC:jl